regulation of lymphotoxin A production [GO:0032681] (BP) Subtypes: negative regulation of lymphotoxin A production [GO:0032721], positive regulation of lymphotoxin A production [GO:0032761] Also known as: regulation of LTA production, regulation of TNF-beta production, regulation of lymphotoxin-alpha production, regulation of tumor necrosis factor-beta production, regulation of lymphotoxin A biosynthetic process Definition: Any process that modulates the frequency, rate, or extent of lymphotoxin A production. Relationships: is a type of regulation of protein metabolic process [GO:0051246]; is a type of GO:1903555; regulates lymphotoxin A production [GO:0032641] Sources: GOC:mah